{
  "gene": "UniProtKB:O14684",
  "gene_name": "Prostaglandin E synthase",
  "term_label": "prostaglandin biosynthetic process",
  "term_id": "GO:0001516",
  "gene_symbol": "PTGES"
}